{
  "gene_name": "Secernin-3",
  "gene": "UniProtKB:Q0VDG4",
  "gene_symbol": "SCRN3",
  "term_id": "UNKNOWN:0002",
  "term_label": "Unknown biological process"
}